{
  "term_label": "regulation of Notch signaling pathway",
  "gene_name": "Lethal(2) giant larvae protein homolog 1",
  "gene": "UniProtKB:Q15334",
  "term_id": "GO:0008593",
  "gene_symbol": "LLGL1"
}